{
  "gene": "UniProtKB:A6QL64",
  "gene_name": "Ankyrin repeat domain-containing protein 36A",
  "term_label": "Unknown molecular function",
  "term_id": "UNKNOWN:0001",
  "gene_symbol": "ANKRD36"
}